{
  "gene_symbol": "DCDC2",
  "term_id": "GO:0001764",
  "gene_name": "Doublecortin domain-containing protein 2",
  "gene": "UniProtKB:Q9UHG0",
  "term_label": "neuron migration"
}